{
  "gene": "UniProtKB:P11142",
  "term_id": "GO:0044183",
  "gene_symbol": "HSPA8",
  "term_label": "protein folding chaperone",
  "gene_name": "Heat shock cognate 71 kDa protein"
}